{
  "gene": "UniProtKB:P63302",
  "gene_symbol": "SELENOW",
  "term_id": "GO:0005829",
  "term_label": "cytosol",
  "gene_name": "Selenoprotein W"
}